{
  "gene_symbol": "NUDT13",
  "term_id": "UNKNOWN:0001",
  "gene": "UniProtKB:Q86X67",
  "term_label": "Unknown molecular function",
  "gene_name": "NAD(P)H pyrophosphatase NUDT13, mitochondrial"
}